{
  "gene_symbol": "PDIK1L",
  "gene": "UniProtKB:Q8N165",
  "gene_name": "Serine_threonine-protein kinase PDIK1L",
  "term_label": "nucleus",
  "term_id": "GO:0005634"
}